{
  "gene_name": "Protein Abitram",
  "gene": "UniProtKB:Q9NX38",
  "term_label": "nucleus",
  "term_id": "GO:0005634",
  "gene_symbol": "ABITRAM"
}